{
  "term_id": "GO:0004842",
  "gene_symbol": "MARCHF2",
  "term_label": "ubiquitin-protein transferase activity",
  "gene_name": "E3 ubiquitin-protein ligase MARCHF2",
  "gene": "UniProtKB:Q9P0N8"
}